{
  "term_id": "GO:1990166",
  "gene_name": "SMC5-SMC6 complex localization factor protein 2",
  "gene": "UniProtKB:Q8IX21",
  "term_label": "protein localization to site of double-strand break",
  "gene_symbol": "SLF2"
}